{
  "gene_symbol": "IGHV3-13",
  "term_id": "UNKNOWN:0003",
  "gene_name": "Immunoglobulin heavy variable 3-13",
  "gene": "UniProtKB:P01766",
  "term_label": "Unknown cellular component"
}